regulation of postsynaptic density protein 95 clustering [GO:1902897] (BP) Definition: Any process that modulates the frequency, rate or extent of postsynaptic density protein 95 clustering. References: PMID:10570482 Sources: GOC:TermGenie, GOC:als, GO_REF:0000058 Relationships: is a type of regulation of protein localization to membrane [GO:1905475]; is a type of GO:1905874; regulates GO:0097119 Also known as: regulation of Dlg4 clustering, regulation of PSD-95 clustering, regulation of post-synaptic density protein 95 clustering